{
  "term_label": "plasma membrane",
  "gene": "UniProtKB:P25092",
  "term_id": "GO:0005886",
  "gene_name": "Guanylyl cyclase C",
  "gene_symbol": "GUCY2C"
}